cellular response to interferon-beta [GO:0035458] (biological process) Relationships: is a type of response to interferon-beta [GO:0035456]; is a type of cellular response to cytokine stimulus [GO:0071345] Also known as: cellular response to fiblaferon, cellular response to fibroblast interferon, cellular response to beta-1 interferon Sources: GOC:sl Definition: Any process that results in a change in state or activity of a cell (in terms of movement, secretion, enzyme production, gene expression, etc.) as a result of an interferon-beta stimulus. Interferon-beta is a type I interferon.